host cytoskeleton [GO:0044163] (cellular component) Subtypes: GO:0120148 Relationships: is_a host intracellular organelle [GO:0033647] Definition: A cellular structure that forms the internal framework of eukaryotic and prokaryotic host cells. The cytoskeleton includes intermediate filaments, microfilaments, microtubules, the microtrabecular lattice, and other structures characterized by a polymeric filamentous nature and long-range order within the cell. The various elements of the cytoskeleton not only serve in the maintenance of cellular shape but also have roles in other cellular functions, including cellular movement, cell division, endocytosis, and movement of organelles. Sources: GOC:rph